{
  "gene_name": "Vascular endothelial growth factor receptor 1",
  "term_id": "GO:0048010",
  "gene_symbol": "FLT1",
  "term_label": "vascular endothelial growth factor receptor signaling pathway",
  "gene": "UniProtKB:P17948"
}